{
  "term_id": "GO:0004479",
  "gene_name": "Methionyl-tRNA formyltransferase, mitochondrial",
  "gene_symbol": "MTFMT",
  "term_label": "methionyl-tRNA formyltransferase activity",
  "gene": "UniProtKB:Q96DP5"
}